{
  "gene_symbol": "CYP4F11",
  "term_label": "arachidonate metabolic process",
  "term_id": "GO:0019369",
  "gene_name": "Cytochrome P450 4F11",
  "gene": "UniProtKB:Q9HBI6"
}